{
  "term_id": "GO:0009986",
  "gene_symbol": "KLRC2",
  "term_label": "cell surface",
  "gene_name": "NKG2-C type II integral membrane protein",
  "gene": "UniProtKB:P26717"
}